regulation of synaptic vesicle lumen acidification [GO:1901546] (biological process) Sources: GOC:TermGenie Also known as: regulation of synaptic vesicle lumen pH reduction, regulation of synaptic vesicle lumen proton loading Relationships: is a type of regulation of proton transport [GO:0010155]; regulates synaptic vesicle lumen acidification [GO:0097401] Definition: Any process that modulates the frequency, rate or extent of synaptic vesicle lumen acidification. Subtypes: negative regulation of synaptic vesicle lumen acidification [GO:1901547], positive regulation of synaptic vesicle lumen acidification [GO:1901548]